{
  "term_label": "placenta development",
  "gene": "UniProtKB:Q86TG7",
  "gene_symbol": "PEG10",
  "gene_name": "Retrotransposon-derived protein PEG10",
  "term_id": "GO:0001890"
}